{
  "term_id": "GO:0032991",
  "gene": "UniProtKB:Q58FF7",
  "term_label": "protein-containing complex",
  "gene_name": "Putative heat shock protein HSP 90-beta-3",
  "gene_symbol": "HSP90AB3P"
}